{
  "gene_symbol": "DNAI3",
  "term_id": "GO:0060294",
  "gene_name": "Dynein axonemal intermediate chain 3",
  "term_label": "cilium movement involved in cell motility",
  "gene": "UniProtKB:Q8IWG1"
}